{
  "term_label": "protein O-linked glycosylation",
  "gene_symbol": "GALNT18",
  "gene_name": "Polypeptide N-acetylgalactosaminyltransferase 18",
  "gene": "UniProtKB:Q6P9A2",
  "term_id": "GO:0006493"
}